negative regulation of formin-nucleated actin cable assembly [GO:0090339] (biological process) Relationships: is a type of negative regulation of actin filament bundle assembly [GO:0032232]; is a type of GO:0090337; negatively regulates formin-nucleated actin cable assembly [GO:0070649] Definition: Any process that decreases the rate, frequency, or extent of formin-nucleated actin cable assembly. Formin-nucleated actin cable assembly is the aggregation, arrangement and bonding together of a set of components to form a formin-nucleated actin cable. A formin-nucleated actin cable is an actin filament bundle that consists of short filaments organized into bundles of uniform polarity, and is nucleated by formins. References: PMID:12810699, PMID:15923184 Sources: GOC:jh, GOC:tb